{
  "term_id": "GO:0005813",
  "gene_symbol": "C10orf90",
  "term_label": "centrosome",
  "gene_name": "(E2-independent) E3 ubiquitin-conjugating enzyme FATS",
  "gene": "UniProtKB:Q96M02"
}